phytoene biosynthetic process [GO:1901174] (biological process) Also known as: phytoene anabolism, phytoene biosynthesis, phytoene formation, phytoene synthesis Definition: The chemical reactions and pathways resulting in the formation of phytoene. Relationships: is a type of carotene biosynthetic process [GO:0016120] Sources: GOC:TermGenie, GOC:yaf, UniPathway:UPA00799